{
  "gene": "UniProtKB:A6NMB9",
  "term_id": "GO:0008568",
  "term_label": "microtubule severing ATPase activity",
  "gene_symbol": "FIGNL2",
  "gene_name": "Fidgetin-like protein 2"
}